{
  "term_label": "oxygen carrier activity",
  "gene_name": "Hemoglobin subunit zeta",
  "gene": "UniProtKB:P02008",
  "term_id": "GO:0005344",
  "gene_symbol": "HBZ"
}